{
  "term_label": "heterochromatin",
  "gene": "UniProtKB:Q99549",
  "term_id": "GO:0000792",
  "gene_symbol": "MPHOSPH8",
  "gene_name": "M-phase phosphoprotein 8"
}